negative regulation of apoptotic process involved in metanephric collecting duct development [GO:1900215] (biological process) References: PMID:17314325 Sources: GOC:TermGenie, GOC:mtg_kidney_jan10, GOC:yaf Definition: Any process that stops, prevents or reduces the frequency, rate or extent of apoptotic process involved in metanephric collecting duct development. Also known as: down regulation of apoptotic cell death of metanephric collecting duct development, down regulation of apoptotic process involved in metanephric collecting duct development, down regulation of apoptotic process of metanephric collecting duct development, down regulation of apoptotic programmed cell death of metanephric collecting duct development, down regulation of programmed cell death by apoptosis of metanephric collecting duct development, down-regulation of apoptotic cell death of metanephric collecting duct development, down-regulation of apoptotic process involved in metanephric collecting duct development, down-regulation of apoptotic process of metanephric collecting duct development, down-regulation of apoptotic programmed cell death of metanephric collecting duct development, down-regulation of programmed cell death by apoptosis of metanephric collecting duct development, downregulation of apoptotic cell death of metanephric collecting duct development, downregulation of apoptotic process involved in metanephric collecting duct development, downregulation of apoptotic process of metanephric collecting duct development, downregulation of apoptotic programmed cell death of metanephric collecting duct development, downregulation of programmed cell death by apoptosis of metanephric collecting duct development, inhibition of apoptotic cell death of metanephric collecting duct development, inhibition of apoptotic process of metanephric collecting duct development, inhibition of apoptotic programmed cell death of metanephric collecting duct development, inhibition of programmed cell death by apoptosis of metanephric collecting duct development, negative regulation of apoptotic cell death of metanephric collecting duct development, negative regulation of apoptotic process of metanephric collecting duct development, negative regulation of apoptotic programmed cell death of metanephric collecting duct development, negative regulation of programmed cell death by apoptosis of metanephric collecting duct development, down regulation of apoptosis of metanephric collecting duct development, down regulation of apoptotic program of metanephric collecting duct development, down regulation of type I programmed cell death of metanephric collecting duct development, down-regulation of apoptosis of metanephric collecting duct development, down-regulation of apoptotic program of metanephric collecting duct development, down-regulation of type I programmed cell death of metanephric collecting duct development, downregulation of apoptosis of metanephric collecting duct development, downregulation of apoptotic program of metanephric collecting duct development, downregulation of type I programmed cell death of metanephric collecting duct development, inhibition of apoptosis of metanephric collecting duct development, inhibition of apoptotic process involved in metanephric collecting duct development, inhibition of apoptotic program of metanephric collecting duct development, inhibition of type I programmed cell death of metanephric collecting duct development, negative regulation of apoptosis of metanephric collecting duct development, negative regulation of apoptotic program of metanephric collecting duct development, negative regulation of type I programmed cell death of metanephric collecting duct development, down regulation of signaling (initiator) caspase activity of metanephric collecting duct development, down-regulation of signaling (initiator) caspase activity of metanephric collecting duct development, downregulation of signaling (initiator) caspase activity of metanephric collecting duct development, inhibition of signaling (initiator) caspase activity of metanephric collecting duct development, negative regulation of signaling (initiator) caspase activity of metanephric collecting duct development Relationships: is a type of regulation of apoptotic process involved in metanephric collecting duct development [GO:1900214]; is a type of negative regulation of apoptotic process involved in development [GO:1904746]; negatively regulates apoptotic process involved in metanephric collecting duct development [GO:1900204]